{
  "term_label": "plasma membrane",
  "term_id": "GO:0005886",
  "gene": "UniProtKB:Q86XP1",
  "gene_name": "Diacylglycerol kinase eta",
  "gene_symbol": "DGKH"
}